{
  "gene_name": "Mothers against decapentaplegic homolog 9",
  "term_label": "SMAD protein signal transduction",
  "gene_symbol": "SMAD9",
  "gene": "UniProtKB:O15198",
  "term_id": "GO:0060395"
}